mannitol transmembrane transport [GO:0015797] (biological process) Also known as: mannitol transport Sources: GOC:ai Relationships: is a type of polyol transmembrane transport [GO:0015791]; is a type of carbohydrate transmembrane transport [GO:0034219] Definition: The directed movement of mannitol across a membrane. Mannitol is the alditol derived from D-mannose by reduction of the aldehyde group.